{
  "gene_name": "Rho guanine nucleotide exchange factor 9",
  "term_id": "GO:0005085",
  "gene_symbol": "ARHGEF9",
  "term_label": "guanyl-nucleotide exchange factor activity",
  "gene": "UniProtKB:O43307"
}